{
  "term_id": "GO:0000981",
  "term_label": "DNA-binding transcription factor activity, RNA polymerase II-specific",
  "gene_symbol": "RLF",
  "gene_name": "Zinc finger protein Rlf",
  "gene": "UniProtKB:Q13129"
}